phenylacetyl-coenzyme A:glycine N-acyltransferase activity [GO:0102080] (molecular function) Sources: EC:2.3.1.192, GOC:pz Definition: Catalysis of the reaction: phenylacetyl-CoA + glycine = H+ + phenylacetylglycine + coenzyme A. Relationships: is a type of acyltransferase activity, transferring groups other than amino-acyl groups [GO:0016747]